{
  "term_label": "DNA binding",
  "gene_symbol": "H2BC13",
  "gene_name": "Histone H2B type 1-L",
  "term_id": "GO:0003677",
  "gene": "UniProtKB:Q99880"
}